target-directed miRNA degradation [GO:0140958] (biological process) Relationships: is a type of miRNA catabolic process [GO:0010587]; is a type of GO:0016441; is a type of negative regulation of miRNA-mediated gene silencing [GO:0060965] Also known as: TDMD, target-directed microRNA degradation References: PMID:33184237, PMID:36150386 Definition: The process in which a miRNA is targeted for degradation by a non-coding RNA or mRNA. The binding of an RNA to a target miRNA within a RISC complex results in either ubiquitin-mediated degradation of AGO protein or the displacement of the 3' end of the miRNA, exposing it to nucleases.